{
  "gene_symbol": "MRPL28",
  "gene_name": "Large ribosomal subunit protein bL28m",
  "term_label": "mitochondrial large ribosomal subunit",
  "term_id": "GO:0005762",
  "gene": "UniProtKB:Q13084"
}